{
  "term_id": "GO:0046359",
  "gene_name": "Short-chain specific acyl-CoA dehydrogenase, mitochondrial",
  "gene_symbol": "ACADS",
  "gene": "UniProtKB:P16219",
  "term_label": "butyrate catabolic process"
}